poly-beta-1,6-N-acetyl-D-glucosamine transmembrane transporter activity [GO:1901515] (molecular function) Definition: Enables the transfer of poly-beta-1,6-N-acetyl-D-glucosamine from one side of a membrane to the other. References: PMID:15090514, PMID:18359807 Sources: GOC:TermGenie Relationships: is a type of GO:0022857